{
  "gene_name": "Dolichol-phosphate mannosyltransferase subunit 1",
  "term_id": "GO:0006488",
  "gene_symbol": "DPM1",
  "term_label": "dolichol-linked oligosaccharide biosynthetic process",
  "gene": "UniProtKB:O60762"
}